heat generation [GO:0031649] (biological process) Subtypes: fever generation [GO:0001660] Relationships: is a type of GO:0001659 Definition: Any homeostatic process in which an organism produces heat, thereby raising its internal temperature. Regulation: regulated by regulation of heat generation [GO:0031650]; negatively regulated by negative regulation of heat generation [GO:0031651]; positively regulated by positive regulation of heat generation [GO:0031652] Sources: GOC:mah